{
  "term_label": "RNA binding",
  "term_id": "GO:0003723",
  "gene_name": "Probable helicase senataxin",
  "gene_symbol": "SETX",
  "gene": "UniProtKB:Q7Z333"
}